{
  "gene_symbol": "EXOC7",
  "term_id": "UNKNOWN:0001",
  "gene": "UniProtKB:Q9UPT5",
  "gene_name": "Exocyst complex component 7",
  "term_label": "Unknown molecular function"
}